{
  "gene_symbol": "OSCP1",
  "term_label": "cytoplasm",
  "gene_name": "Protein OSCP1",
  "gene": "UniProtKB:Q8WVF1",
  "term_id": "GO:0005737"
}